{
  "term_id": "GO:0006979",
  "gene_symbol": "PARK7",
  "gene": "UniProtKB:Q99497",
  "term_label": "response to oxidative stress",
  "gene_name": "Parkinson disease protein 7"
}